{
  "term_id": "GO:0051604",
  "gene_symbol": "CTSG",
  "gene_name": "Cathepsin G",
  "gene": "UniProtKB:P08311",
  "term_label": "protein maturation"
}